positive regulation of endodermal cell differentiation [GO:1903226] (biological process) References: PMID:23154389 Sources: GOC:TermGenie, GOC:als, GO_REF:0000058 Relationships: is a type of GO:0045597; is a type of regulation of endodermal cell differentiation [GO:1903224]; positively regulates GO:0035987 Definition: Any process that activates or increases the frequency, rate or extent of endodermal cell differentiation. Also known as: positive regulation of endoderm cell differentiation, up regulation of endoderm cell differentiation, up regulation of endodermal cell differentiation, up-regulation of endoderm cell differentiation, up-regulation of endodermal cell differentiation, upregulation of endoderm cell differentiation, upregulation of endodermal cell differentiation, activation of endoderm cell differentiation, activation of endodermal cell differentiation